{
  "gene_symbol": "ZNF503",
  "gene_name": "Zinc finger protein 503",
  "gene": "UniProtKB:Q96F45",
  "term_id": "GO:0045892",
  "term_label": "negative regulation of DNA-templated transcription"
}